{
  "term_label": "ubiquitin binding",
  "gene_name": "Vacuolar protein-sorting-associated protein 36",
  "term_id": "GO:0043130",
  "gene": "UniProtKB:Q86VN1",
  "gene_symbol": "VPS36"
}